{
  "term_id": "GO:0047429",
  "gene": "UniProtKB:O14638",
  "term_label": "nucleoside triphosphate diphosphatase activity",
  "gene_symbol": "ENPP3",
  "gene_name": "Ectonucleotide pyrophosphatase_phosphodiesterase family member 3"
}